{
  "gene": "UniProtKB:Q2VWP7",
  "gene_symbol": "PRTG",
  "term_id": "UNKNOWN:0003",
  "term_label": "Unknown cellular component",
  "gene_name": "Protogenin"
}